TFIIIA-class transcription factor binding [GO:0001155] (molecular function) Relationships: is a type of RNA polymerase III general transcription initiation factor binding [GO:0001025] Definition: Binding to an RNA polymerase III transcription factor of the TFIIIA class, one of the factors involved in formation of the preinitiation complex (PIC) at RNA polymerase III promoters. References: PMID:12381659 Sources: GOC:txnOH